endoplasmic reticulum-plasma membrane contact site [GO:0140268] (cellular component) Relationships: is a type of organelle membrane contact site [GO:0044232] Also known as: EPCS, ER-PM contact site, ER-plasma membrane contact site, endoplasmic reticulum-plasma membrane contact junction Definition: A contact site between the endoplasmic reticulum membrane and the plasma membrane, structured by bridging complexes. References: PMID:23041194, PMID:27955928, PMID:29290560, PMID:29782498, PMID:30012696